seed maturation [GO:0010431] (biological process) Definition: A process in seed development that occurs after embryogenesis by which a quiescent state is established in a seed. Seed maturation is characterized by storage compound accumulation, acquisition of desiccation tolerance, growth arrest and the entry into a dormancy period of variable length that is broken upon germination. References: PMID:16096971 Relationships: is a type of developmental process involved in reproduction [GO:0003006]; is a type of developmental maturation [GO:0021700]; is a type of multicellular organismal reproductive process [GO:0048609]; is part of seed development [GO:0048316] Regulation: regulated by regulation of seed maturation [GO:2000034]; negatively regulated by GO:2000692; positively regulated by positive regulation of seed maturation [GO:2000693]